{
  "gene_name": "Nucleotide sugar transporter SLC35B4",
  "gene_symbol": "SLC35B4",
  "term_id": "GO:0005464",
  "term_label": "UDP-xylose transmembrane transporter activity",
  "gene": "UniProtKB:Q969S0"
}